{
  "gene_symbol": "RPP38",
  "term_label": "tRNA 5'-leader removal",
  "gene_name": "Ribonuclease P protein subunit p38",
  "gene": "UniProtKB:P78345",
  "term_id": "GO:0001682"
}